{
  "gene_symbol": "DCAF11",
  "term_label": "proteasome-mediated ubiquitin-dependent protein catabolic process",
  "term_id": "GO:0043161",
  "gene_name": "DDB1- and CUL4-associated factor 11",
  "gene": "UniProtKB:Q8TEB1"
}